Toll-like receptor binding [GO:0035325] (molecular function) Subtypes: GO:0035662, Toll-like receptor 2 binding [GO:0035663] References: PMID:19076341 Relationships: is a type of signaling receptor binding [GO:0005102] Also known as: TLR binding Definition: Binding to a Toll-like protein, a pattern recognition receptor that binds pattern motifs from a variety of microbial sources to initiate an innate immune response.